{
  "term_id": "GO:0030154",
  "gene": "UniProtKB:P84022",
  "gene_name": "Mothers against decapentaplegic homolog 3",
  "gene_symbol": "SMAD3",
  "term_label": "cell differentiation"
}